{
  "gene_symbol": "PRPS2",
  "term_id": "GO:0005737",
  "gene_name": "Ribose-phosphate pyrophosphokinase 2",
  "term_label": "cytoplasm",
  "gene": "UniProtKB:P11908"
}